synaptic vesicle recycling [GO:0036465] (biological process) Also known as: kiss-and-run synaptic vesicle recycling, kiss-and-stay synaptic vesicle recycling References: PMID:15217342, PMID:22026965, PMID:23245563 Sources: GOC:PARL, GOC:bf, GOC:pad Subtypes: synaptic vesicle recycling via endosome [GO:0036466] Relationships: is a type of transport [GO:0006810]; is a type of GO:0051649; BFO_0000050 synaptic vesicle cycle [GO:0099504] Definition: The trafficking of synaptic vesicles from the pre-synaptic membrane so the vesicle can dock and prime for another round of exocytosis and neurotransmitter release. Recycling occurs after synaptic vesicle exocytosis, and is necessary to replenish presynaptic vesicle pools, sustain transmitter release and preserve the structural integrity of the presynaptic membrane. Recycling can occur following transient fusion with the presynaptic membrane (kiss and run), or via endocytosis of presynaptic membrane. Regulation: regulated by GO:1903421; negatively regulated by negative regulation of synaptic vesicle recycling [GO:1903422]; positively regulated by GO:1903423